{
  "gene": "UniProtKB:O15400",
  "gene_name": "Syntaxin-7",
  "term_id": "GO:0008021",
  "gene_symbol": "STX7",
  "term_label": "synaptic vesicle"
}